regulation of nucleus size [GO:0097298] (biological process) References: PMID:19366728 Sources: GOC:al, GOC:mah Also known as: regulation of nuclear size, regulation of nuclear volume Relationships: is a type of regulation of cellular component size [GO:0032535] Definition: Any process that modulates the size of the nucleus.